adrenal cortex formation [GO:0035802] (biological process) Also known as: adrenal gland cortex formation References: PMID:12185666, PMID:21115154 Relationships: is_a anatomical structure formation involved in morphogenesis [GO:0048646]; is part of adrenal cortex development [GO:0035801] Definition: The process that gives rise to the adrenal cortex. This process pertains to the initial formation of a structure from unspecified parts. The adrenogonadal primordium from which the adrenal cortex is formed derives from a condensation of coelomic epithelial cells (the urogenital ridge; the same structure from which gonads and kidney also originate).